negative regulation of attachment of mitotic spindle microtubules to kinetochore [GO:1902424] (biological process) Definition: Any process that stops, prevents or reduces the frequency, rate or extent of attachment of spindle microtubules to kinetochore involved in mitotic sister chromatid segregation. References: PMID:22065639 Sources: GOC:TermGenie, GOC:vw Also known as: down regulation of attachment of spindle microtubules to kinetochore involved in mitosis, down regulation of attachment of spindle microtubules to kinetochore involved in mitotic sister chromatid segregation, down regulation of attachment of spindle microtubules to mitotic chromosome, down-regulation of attachment of spindle microtubules to kinetochore involved in mitosis, down-regulation of attachment of spindle microtubules to kinetochore involved in mitotic sister chromatid segregation, down-regulation of attachment of spindle microtubules to mitotic chromosome, downregulation of attachment of spindle microtubules to kinetochore involved in mitosis, downregulation of attachment of spindle microtubules to kinetochore involved in mitotic sister chromatid segregation, downregulation of attachment of spindle microtubules to mitotic chromosome, negative regulation of attachment of spindle microtubules to kinetochore involved in mitosis, negative regulation of attachment of spindle microtubules to kinetochore involved in mitotic sister chromatid segregation, negative regulation of attachment of spindle microtubules to mitotic chromosome, negative regulation of mitotic attachment of spindle microtubules to kinetochore, inhibition of attachment of spindle microtubules to kinetochore involved in mitosis, inhibition of attachment of spindle microtubules to kinetochore involved in mitotic sister chromatid segregation, inhibition of attachment of spindle microtubules to mitotic chromosome, down regulation of attachment of spindle microtubules to kinetochore during mitosis, down regulation of mitotic bipolar attachment, down-regulation of attachment of spindle microtubules to kinetochore during mitosis, down-regulation of mitotic bipolar attachment, downregulation of attachment of spindle microtubules to kinetochore during mitosis, downregulation of mitotic bipolar attachment, inhibition of attachment of spindle microtubules to kinetochore during mitosis, inhibition of mitotic bipolar attachment, negative regulation of attachment of spindle microtubules to kinetochore during mitosis, negative regulation of mitotic bipolar attachment Relationships: is a type of negative regulation of attachment of spindle microtubules to kinetochore [GO:0051986]; is a type of GO:1902423; negatively regulates GO:0051315